{
  "gene_symbol": "KPRP",
  "gene_name": "Keratinocyte proline-rich protein",
  "gene": "UniProtKB:Q5T749",
  "term_label": "Unknown molecular function",
  "term_id": "UNKNOWN:0001"
}